{
  "gene": "UniProtKB:Q9H2X6",
  "term_id": "GO:0003714",
  "gene_name": "Homeodomain-interacting protein kinase 2",
  "term_label": "transcription corepressor activity",
  "gene_symbol": "HIPK2"
}